{
  "gene_symbol": "CDC14B",
  "gene": "UniProtKB:O60729",
  "term_label": "spindle pole",
  "gene_name": "Dual specificity protein phosphatase CDC14B",
  "term_id": "GO:0000922"
}